{
  "term_id": "UNKNOWN:0003",
  "gene_name": "Protein phosphatase 1L",
  "gene": "UniProtKB:Q5SGD2",
  "gene_symbol": "PPM1L",
  "term_label": "Unknown cellular component"
}